D-aspartate oxidase activity [GO:0008445] (molecular function) Sources: RHEA:12512 Relationships: is a type of D-amino-acid oxidase activity [GO:0003884] Also known as: D-aspartate:oxygen oxidoreductase (deaminating), D-aspartic oxidase activity, aspartic oxidase activity Definition: Catalysis of the reaction: D-aspartate + H2O + O2 = H2O2 + NH4+ + oxaloacetate.